{
  "gene_symbol": "LINC02901",
  "term_id": "UNKNOWN:0002",
  "gene": "UniProtKB:Q4VX62",
  "gene_name": "Putative uncharacterized protein LINC02901",
  "term_label": "Unknown biological process"
}